{
  "term_label": "cilium",
  "gene": "UniProtKB:Q86UC2",
  "term_id": "GO:0005929",
  "gene_name": "Radial spoke head protein 3 homolog",
  "gene_symbol": "RSPH3"
}